{
  "term_id": "GO:0015630",
  "gene_symbol": "GTSE1",
  "gene": "UniProtKB:Q9NYZ3",
  "term_label": "microtubule cytoskeleton",
  "gene_name": "G2 and S phase-expressed protein 1"
}